negative regulation of transdifferentiation [GO:1903619] (biological process) References: PMID:22118091 Sources: GOC:TermGenie, GO_REF:0000058 Also known as: down regulation of transdifferentiation, down-regulation of transdifferentiation, downregulation of transdifferentiation, inhibition of transdifferentiation Definition: Any process that stops, prevents or reduces the frequency, rate or extent of transdifferentiation. Relationships: is a type of negative regulation of cell differentiation [GO:0045596]; is a type of regulation of transdifferentiation [GO:1903618]; negatively regulates GO:0060290